{
  "gene": "UniProtKB:Q00266",
  "term_label": "S-adenosylmethionine biosynthetic process",
  "gene_symbol": "MAT1A",
  "gene_name": "S-adenosylmethionine synthase isoform type-1",
  "term_id": "GO:0006556"
}